{
  "term_id": "GO:0005737",
  "gene_name": "Triple functional domain protein",
  "term_label": "cytoplasm",
  "gene_symbol": "TRIO",
  "gene": "UniProtKB:O75962"
}